{
  "gene_symbol": "HTR3D",
  "term_id": "GO:0005231",
  "gene": "UniProtKB:Q70Z44",
  "gene_name": "5-hydroxytryptamine receptor 3D",
  "term_label": "excitatory extracellular ligand-gated monoatomic ion channel activity"
}